{
  "term_id": "UNKNOWN:0003",
  "gene_name": "G antigen 10",
  "term_label": "Unknown cellular component",
  "gene": "UniProtKB:A6NGK3",
  "gene_symbol": "GAGE10"
}